{
  "term_id": "GO:0008327",
  "gene_name": "Methyl-CpG-binding domain protein 3-like 2",
  "gene_symbol": "MBD3L2",
  "gene": "UniProtKB:Q8NHZ7",
  "term_label": "methyl-CpG binding"
}